{
  "term_label": "nucleus",
  "term_id": "GO:0005634",
  "gene": "UniProtKB:Q96KN3",
  "gene_name": "Homeobox protein PKNOX2",
  "gene_symbol": "PKNOX2"
}